type II interferon-mediated signaling pathway [GO:0060333] (biological process) Relationships: is a type of interferon-mediated signaling pathway [GO:0140888]; is part of cellular response to type II interferon [GO:0071346] References: PMID:28901902 Sources: GOC:add, GOC:dph, GOC:signaling Also known as: gamma-interferon-mediated signaling pathway, immune interferon signaling pathway, interferon-gamma-mediated signaling pathway, interferon-gamma-mediated signalling pathway, type II IFN-mediated signaling pathway Regulation: regulated by regulation of type II interferon-mediated signaling pathway [GO:0060334]; positively regulated by positive regulation of type II interferon-mediated signaling pathway [GO:0060335]; negatively regulated by negative regulation of type II interferon-mediated signaling pathway [GO:0060336] Definition: The series of molecular signals initiated by interferon-gamma binding to its receptor on the surface of a target cell, and ending with the regulation of a downstream cellular process, e.g. transcription. Interferon gamma is the only member of the type II interferon found so far.